{
  "gene": "UniProtKB:A5X5Y0",
  "gene_name": "5-hydroxytryptamine receptor 3E",
  "term_id": "GO:0045202",
  "gene_symbol": "HTR3E",
  "term_label": "synapse"
}